{
  "gene": "UniProtKB:Q5MNZ6",
  "term_label": "phosphatidylinositol-3,5-bisphosphate binding",
  "gene_name": "WD repeat domain phosphoinositide-interacting protein 3",
  "gene_symbol": "WDR45B",
  "term_id": "GO:0080025"
}